DNA-binding transcription factor activity, RNA polymerase II-specific [GO:0000981] (molecular function) Note: For usage guidance, see comment in GO:0003700 ; DNA-binding transcription factor activity. Definition: A DNA-binding transcription factor activity that modulates the transcription of specific gene sets transcribed by RNA polymerase II. Subtypes: DNA-binding transcription repressor activity, RNA polymerase II-specific [GO:0001227], DNA-binding transcription activator activity, RNA polymerase II-specific [GO:0001228], nuclear receptor activity [GO:0004879] Relationships: is a type of DNA-binding transcription factor activity [GO:0003700]; is part of regulation of transcription by RNA polymerase II [GO:0006357]; BFO_0000051 RNA polymerase II transcription regulatory region sequence-specific DNA binding [GO:0000977]; occurs in chromatin [GO:0000785] Sources: GOC:txnOH-2018 Also known as: transcription factor, RNA polymerase II transcription factor activity, sequence-specific DNA binding, RNA polymerase II transcription factor activity, sequence-specific transcription regulatory region DNA binding, sequence-specific DNA binding RNA polymerase II transcription factor activity, RNA polymerase II core promoter proximal region sequence-specific DNA binding transcription factor activity, RNA polymerase II distal enhancer sequence-specific DNA binding transcription factor activity, RNA polymerase II transcription factor activity, copper ion regulated core promoter proximal region sequence-specific binding, RNA polymerase II transcription factor activity, copper ion regulated proximal promoter sequence-specific DNA binding, RNA polymerase II transcription factor activity, metal ion regulated core promoter proximal region sequence-specific binding, RNA polymerase II transcription factor activity, metal ion regulated proximal promoter sequence-specific DNA binding, RNA polymerase II transcription factor activity, metal ion regulated sequence-specific DNA binding, RNA polymerase II transcription factor activity, zinc ion regulated core promoter proximal region sequence-specific DNA binding, RNA polymerase II transcription factor activity, zinc ion regulated proximal promoter sequence-specific DNA binding, copper ion regulated core promoter proximal region sequence-specific DNA binding RNA polymerase II transcription factor activity, metal ion regulated core promoter proximal region sequence-specific DNA binding RNA polymerase II transcription factor activity, metal ion regulated sequence-specific DNA binding RNA polymerase II transcription factor activity, sequence-specific distal enhancer binding RNA polymerase II transcription factor activity, transcription factor activity, RNA polymerase II core promoter proximal region sequence-specific binding, transcription factor activity, RNA polymerase II distal enhancer sequence-specific binding, transcription factor activity, RNA polymerase II proximal promoter sequence-specific DNA binding, zinc ion regulated core promoter proximal region sequence-specific DNA binding RNA polymerase II transcription factor activity, sequence-specific transcription regulatory region DNA binding RNA polymerase II transcription factor recruiting transcription factor activity